{
  "term_id": "GO:0006955",
  "gene_symbol": "IGLV3-21",
  "term_label": "immune response",
  "gene_name": "Immunoglobulin lambda variable 3-21",
  "gene": "UniProtKB:P80748"
}